{
  "gene_name": "Transcriptional repressor scratch 1",
  "gene": "UniProtKB:Q9BWW7",
  "term_label": "RNA polymerase II cis-regulatory region sequence-specific DNA binding",
  "gene_symbol": "SCRT1",
  "term_id": "GO:0000978"
}